rhombomere boundary formation [GO:0021654] (biological process) Definition: The process that gives rise to a rhombomere boundary. This process pertains to the initial formation of a boundary delimiting a rhombomere. Rhombomeres are transverse segments of the developing rhombencephalon that are lineage restricted, express different genes from one another, and adopt different developmental fates. Rhombomeres are numbered in anterior to posterior order. Sources: GOC:cls, GOC:dgh, GOC:dph, GOC:jid, GO_REF:0000021 Relationships: is a type of formation of anatomical boundary [GO:0048859]; is part of rhombomere formation [GO:0021594]